{
  "gene_symbol": "KLHL38",
  "term_label": "proteasome-mediated ubiquitin-dependent protein catabolic process",
  "term_id": "GO:0043161",
  "gene": "UniProtKB:Q2WGJ6",
  "gene_name": "Kelch-like protein 38"
}